{
  "gene_symbol": "GRK6",
  "term_label": "cytoplasm",
  "gene_name": "G protein-coupled receptor kinase 6",
  "gene": "UniProtKB:P43250",
  "term_id": "GO:0005737"
}